actin filament bundle assembly [GO:0051017] (biological process) Sources: GOC:ai Relationships: is a type of cellular component assembly [GO:0022607]; is a type of actin filament bundle organization [GO:0061572] Also known as: actin bundling activity, actin cable assembly, actin cable formation Regulation: regulated by regulation of actin filament bundle assembly [GO:0032231]; negatively regulated by negative regulation of actin filament bundle assembly [GO:0032232]; positively regulated by GO:0032233 Definition: The assembly of actin filament bundles; actin filaments are on the same axis but may be oriented with the same or opposite polarities and may be packed with different levels of tightness. Subtypes: contractile actin filament bundle assembly [GO:0030038], parallel actin filament bundle assembly [GO:0030046], actin rod assembly [GO:0031247], actomyosin contractile ring actin filament bundle assembly [GO:0071519]